{
  "gene_symbol": "GATAD2A",
  "term_id": "GO:0006338",
  "gene": "UniProtKB:Q86YP4",
  "term_label": "chromatin remodeling",
  "gene_name": "Transcriptional repressor p66-alpha"
}